{
  "term_label": "positive regulation of cell migration",
  "term_id": "GO:0030335",
  "gene": "UniProtKB:Q13591",
  "gene_symbol": "SEMA5A",
  "gene_name": "Semaphorin-5A"
}